BH2 domain binding [GO:0051433] (molecular function) References: PMID:11048732, PMID:12133724, PMID:9020082, PMID:9704409 Sources: Prosite:PS01258 Relationships: is a type of BH domain binding [GO:0051400] Definition: Binding to a BH2 protein domain, present in Bcl-2 family members. Proteins that act as inhibitors of apoptosis harbour at least three BH domains: BH1, BH2 and BH3; the BH1 and BH2 domains are found in all death antagonists of the Bcl-2 family but only in one class of death agonists.